RNA nuclease activity [GO:0004540] (molecular function) Relationships: is a type of nuclease activity [GO:0004518]; is a type of catalytic activity, acting on RNA [GO:0140098] Subtypes: RNA endonuclease activity [GO:0004521], RNA exonuclease activity [GO:0004532], tRNA-specific ribonuclease activity [GO:0004549], GO:0032296 Also known as: ribonuclease activity Definition: Catalysis of the cleavage of phosphodiester bonds in chains of RNA. Regulation: RO_0002212 by ribonuclease inhibitor activity [GO:0008428]; regulated by regulation of ribonuclease activity [GO:0060700]; positively regulated by ribonuclease activator activity [GO:0170054] Sources: GOC:mah, ISBN:0198547684